 [go#goslim:mouse] Note: Mouse GO slim